acetate CoA-transferase activity [GO:0008775] (molecular function) Also known as: acetate coenzyme A-transferase activity, acetyl-CoA:acetoacetate CoA transferase activity, acyl-CoA:acetate CoA-transferase activity, butyryl CoA:acetate CoA transferase activity, butyryl coenzyme A transferase activity, succinyl-CoA:acetate CoA transferase activity Sources: EC:2.8.3.8 Relationships: is a type of CoA-transferase activity [GO:0008410] Definition: Catalysis of the reaction: acyl-CoA + acetate = a fatty acid anion + acetyl-CoA.